{
  "gene_symbol": "SEMA7A",
  "gene": "UniProtKB:O75326",
  "gene_name": "Semaphorin-7A",
  "term_id": "GO:0050727",
  "term_label": "regulation of inflammatory response"
}